{
  "gene": "UniProtKB:Q9UMX3",
  "term_label": "extrinsic apoptotic signaling pathway in absence of ligand",
  "gene_name": "Bcl-2-related ovarian killer protein",
  "gene_symbol": "BOK",
  "term_id": "GO:0097192"
}